{
  "gene_name": "Tight junction protein ZO-2",
  "term_label": "cell-cell junction organization",
  "gene": "UniProtKB:Q9UDY2",
  "term_id": "GO:0045216",
  "gene_symbol": "TJP2"
}